{
  "term_id": "GO:0005634",
  "gene_name": "Germ cell-less protein-like 2",
  "gene": "UniProtKB:Q8NEA9",
  "term_label": "nucleus",
  "gene_symbol": "GMCL2"
}